{
  "gene_symbol": "NFATC2IP",
  "term_label": "positive regulation of transcription by RNA polymerase II",
  "term_id": "GO:0045944",
  "gene": "UniProtKB:Q8NCF5",
  "gene_name": "NFATC2-interacting protein"
}